{
  "term_id": "GO:0005085",
  "gene_name": "Ral-GDS-related protein",
  "term_label": "guanyl-nucleotide exchange factor activity",
  "gene": "UniProtKB:Q8IZJ4",
  "gene_symbol": "RGL4"
}